regulation of nitrosative stress-induced intrinsic apoptotic signaling pathway [GO:1905258] (biological process) Definition: Any process that modulates the frequency, rate or extent of intrinsic apoptotic signaling pathway in response to nitrosative stress. References: PMID:14752510 Sources: GOC:PARL, GOC:TermGenie, GOC:bf, GO_REF:0000058 Also known as: regulation of intrinsic apoptotic signaling pathway in response to nitrosative stress, regulation of nitrosative stress-induced apoptosis Relationships: is a type of GO:0080135; is a type of regulation of intrinsic apoptotic signaling pathway [GO:2001242]; regulates intrinsic apoptotic signaling pathway in response to nitrosative stress [GO:1990442] Subtypes: negative regulation of nitrosative stress-induced intrinsic apoptotic signaling pathway [GO:1905259], positive regulation of nitrosative stress-induced intrinsic apoptotic signaling pathway [GO:1905260]